regulation of centromeric sister chromatid cohesion [GO:0070602] (BP) Also known as: regulation of sister chromatid cohesion at centromere Sources: GOC:mah Relationships: is a type of regulation of sister chromatid cohesion [GO:0007063]; regulates centromeric sister chromatid cohesion [GO:0070601] Subtypes: regulation of maintenance of meiotic sister chromatid cohesion, centromeric [GO:2000709], regulation of maintenance of mitotic sister chromatid cohesion, centromeric [GO:2000718] Definition: Any process that modulates the frequency, rate or extent of sister chromatid cohesion in the centromeric region of a chromosome.